{
  "term_id": "GO:0042391",
  "gene_name": "Calcium-activated potassium channel subunit alpha-1",
  "gene_symbol": "KCNMA1",
  "gene": "UniProtKB:Q12791",
  "term_label": "regulation of membrane potential"
}